negative regulation of blood vessel morphogenesis [GO:2000181] (BP) Definition: Any process that stops, prevents, or reduces the frequency, rate or extent of blood vessel morphogenesis. Sources: GOC:dph, GOC:yaf Subtypes: negative regulation of angiogenesis [GO:0016525], negative regulation of testicular blood vessel morphogenesis [GO:0061369], negative regulation of artery morphogenesis [GO:1905652] Relationships: is a type of GO:0022603; is a type of negative regulation of vasculature development [GO:1901343]; negatively regulates blood vessel morphogenesis [GO:0048514]